{
  "gene_symbol": "CAB39L",
  "gene_name": "Calcium-binding protein 39-like",
  "gene": "UniProtKB:Q9H9S4",
  "term_id": "UNKNOWN:0003",
  "term_label": "Unknown cellular component"
}